{
  "gene": "UniProtKB:Q13239",
  "term_label": "COP9 signalosome",
  "gene_name": "Src-like-adapter",
  "term_id": "GO:0008180",
  "gene_symbol": "SLA"
}